{
  "gene": "UniProtKB:A6NJT0",
  "gene_symbol": "UNCX",
  "gene_name": "Homeobox protein unc-4 homolog",
  "term_label": "Unknown cellular component",
  "term_id": "UNKNOWN:0003"
}